{
  "term_label": "cytoplasm",
  "gene": "UniProtKB:P18754",
  "gene_symbol": "RCC1",
  "term_id": "GO:0005737",
  "gene_name": "Regulator of chromosome condensation"
}